sodium:potassium-exchanging ATPase complex [GO:0005890] (cellular component) Sources: ISBN:0198506732 Also known as: sodium pump, sodium/potassium-exchanging ATPase complex Definition: Sodium:potassium-exchanging ATPases are tetrameric proteins, consisting of two large alpha subunits and two smaller beta subunits. The alpha subunits bear the active site and penetrate the membrane, while the beta subunits carry oligosaccharide groups and face the cell exterior. Relationships: is a type of cation-transporting ATPase complex [GO:0090533]; is a type of plasma membrane protein complex [GO:0098797]